septum transversum development [GO:0003343] (biological process) Definition: The progression of the septum transversum from its initial formation to the mature structure. The septum transversum is a portion of the trunk mesenchyme. References: PMID:18722343 Sources: GOC:dph Relationships: is_a mesenchyme development [GO:0060485]